{
  "gene_symbol": "MARCHF8",
  "term_id": "GO:0000209",
  "gene_name": "E3 ubiquitin-protein ligase MARCHF8",
  "term_label": "protein polyubiquitination",
  "gene": "UniProtKB:Q5T0T0"
}